{
  "gene": "UniProtKB:P0DP74",
  "term_label": "chemoattractant activity",
  "gene_symbol": "DEFB130A",
  "term_id": "GO:0042056",
  "gene_name": "Beta-defensin 130A"
}